{
  "term_label": "plasma membrane",
  "gene_symbol": "CFTR",
  "gene": "UniProtKB:P13569",
  "term_id": "GO:0005886",
  "gene_name": "Cystic fibrosis transmembrane conductance regulator"
}